NatA complex [GO:0031415] (cellular component) Definition: A conserved complex that catalyzes the transfer of an acetyl group to an N-terminal Ser, Ala, Gly, or Thr residue of a protein acceptor molecule. In Saccharomyces the complex includes Nat1p and Ard1p, and may contain additional proteins. References: PMID:12890471 Relationships: is a type of N-terminal protein acetyltransferase complex [GO:0031414] Also known as: N-terminal acetyltransferase A complex